histone H3-K14 acetyltransferase complex [GO:0036409] (cellular component) References: PMID:21289066 Sources: GOC:vw Also known as: H3-K14 histone acetyltransferase complex, histone H3 Lys 14 (H3K14) acetyltransferase complex, histone H3K14 acetyltransferase complex, histone acetyltransferase complex (H3-K14 specific) Subtypes: Mst2 histone acetyltransferase complex [GO:0036410] Relationships: is a type of H3 histone acetyltransferase complex [GO:0070775]; is_a GO:0140513 Definition: A protein complex that can catalyze the acetylation of lysine at position 14 in histone H3.